{
  "gene_symbol": "TTC19",
  "gene_name": "Tetratricopeptide repeat protein 19, mitochondrial",
  "term_label": "mitochondrial inner membrane",
  "gene": "UniProtKB:Q6DKK2",
  "term_id": "GO:0005743"
}